{
  "term_label": "Unknown cellular component",
  "gene_symbol": "TMC3",
  "gene_name": "Transmembrane channel-like protein 3",
  "term_id": "UNKNOWN:0003",
  "gene": "UniProtKB:Q7Z5M5"
}